{
  "gene_symbol": "PLK2",
  "gene": "UniProtKB:Q9NYY3",
  "term_label": "G1/S transition of mitotic cell cycle",
  "term_id": "GO:0000082",
  "gene_name": "Serine_threonine-protein kinase PLK2"
}